{
  "gene_name": "RANBP2-like and GRIP domain-containing protein 2",
  "term_label": "NLS-bearing protein import into nucleus",
  "gene_symbol": "RGPD2",
  "term_id": "GO:0006607",
  "gene": "UniProtKB:P0DJD1"
}